{
  "gene_symbol": "RHOG",
  "gene_name": "Rho-related GTP-binding protein RhoG",
  "term_id": "GO:0005525",
  "gene": "UniProtKB:P84095",
  "term_label": "GTP binding"
}